thymidine metabolic process [GO:0046104] (biological process) Definition: The chemical reactions and pathways involving thymidine, deoxyribosylthymine thymine 2-deoxyriboside, a deoxynucleoside very widely distributed but occurring almost entirely as phosphoric esters in deoxynucleotides and deoxyribonucleic acid, DNA. Sources: GOC:go_curators Also known as: deoxyribosylthymine metabolic process, deoxyribosylthymine metabolism, thymidine metabolism Relationships: is a type of pyrimidine deoxyribonucleoside metabolic process [GO:0046125] Subtypes: thymidine catabolic process [GO:0006214], thymidine biosynthetic process [GO:0046105]